protein N-acetyltransferase activity [GO:0034212] (molecular function) Definition: Catalysis of the acetylation of an amino acid residue of a peptide or protein, according to the reaction: acetyl-CoA + peptide = CoA + N-acetylpeptide. Relationships: is a type of N-acetyltransferase activity [GO:0008080]; is a type of protein N-acyltransferase activity [GO:0140186] Subtypes: GO:0004596, protein-lysine-acetyltransferase activity [GO:0061733] Also known as: peptide N-acetyltransferase activity Sources: GOC:mah